{
  "gene_name": "Wee1-like protein kinase",
  "term_label": "cytoplasm",
  "gene_symbol": "WEE1",
  "term_id": "GO:0005737",
  "gene": "UniProtKB:P30291"
}